{
  "gene": "UniProtKB:Q9NZN8",
  "term_id": "GO:0030015",
  "term_label": "CCR4-NOT core complex",
  "gene_symbol": "CNOT2",
  "gene_name": "CCR4-NOT transcription complex subunit 2"
}